phosphatidylinositol-3-phosphate binding [GO:0032266] (molecular function) Relationships: is a type of phosphatidylinositol phosphate binding [GO:1901981] Definition: Binding to phosphatidylinositol-3-phosphate, a derivative of phosphatidylinositol in which the inositol ring is phosphorylated at the 3' position. Also known as: PtdIns-3-P binding, phosphatidylinositol 3-phosphate binding References: PMID:10209156, PMID:11395417, PMID:11557775 Sources: GOC:bf